{
  "term_label": "3'-5'-RNA exonuclease activity",
  "gene_symbol": "ERI1",
  "gene_name": "3'-5' exoribonuclease 1",
  "term_id": "GO:0000175",
  "gene": "UniProtKB:Q8IV48"
}